{
  "term_id": "GO:0001228",
  "gene_symbol": "SOX15",
  "term_label": "DNA-binding transcription activator activity, RNA polymerase II-specific",
  "gene_name": "Protein SOX-15",
  "gene": "UniProtKB:O60248"
}